{
  "gene": "UniProtKB:P05107",
  "term_label": "protein kinase binding",
  "gene_symbol": "ITGB2",
  "term_id": "GO:0019901",
  "gene_name": "Integrin beta-2"
}